{
  "gene_name": "Mismatch repair endonuclease PMS2",
  "gene": "UniProtKB:P54278",
  "gene_symbol": "PMS2",
  "term_id": "GO:0016887",
  "term_label": "ATP hydrolysis activity"
}